{
  "gene_name": "Core histone macro-H2A.1",
  "gene_symbol": "MACROH2A1",
  "term_label": "nucleosome",
  "term_id": "GO:0000786",
  "gene": "UniProtKB:O75367"
}